{
  "term_label": "cytoplasmic exosome (RNase complex)",
  "gene": "UniProtKB:Q9NQT4",
  "term_id": "GO:0000177",
  "gene_symbol": "EXOSC5",
  "gene_name": "Exosome complex component RRP46"
}